Edg-3 sphingosine 1-phosphate receptor binding [GO:0031756] (molecular function) Definition: Binding to an Edg-3 sphingosine 1-phosphate receptor. Also known as: Edg-3 sphingosine 1-phosphate receptor ligand Relationships: is a type of endothelial differentiation G protein-coupled receptor binding [GO:0031753] Sources: GOC:mah, GOC:nln